aerobic cobalamin biosynthetic process [GO:0019250] (BP) Definition: The chemical reactions and pathways resulting in the formation of cobalamin (vitamin B12) in the presence of oxygen. Sources: GOC:go_curators Also known as: aerobic cobalamin anabolism, aerobic cobalamin biosynthesis, aerobic cobalamin formation, aerobic cobalamin synthesis, aerobic vitamin B12 biosynthesis, aerobic vitamin B12 biosynthetic process, cobalamin biosynthesis, aerobic, cobalamin biosynthetic process, aerobic, vitamin B12 biosynthesis, aerobic, vitamin B12 biosynthetic process, aerobic Relationships: is a type of GO:0009236